regulation of androst-4-ene-3,17-dione biosynthetic process [GO:1903454] (biological process) Subtypes: negative regulation of androst-4-ene-3,17-dione biosynthetic process [GO:1903455], positive regulation of androst-4-ene-3,17-dione biosynthetic process [GO:1903456] Relationships: is_a regulation of ketone biosynthetic process [GO:0010566]; is a type of regulation of steroid biosynthetic process [GO:0050810]; regulates androst-4-ene-3,17-dione biosynthetic process [GO:1903449] Definition: Any process that modulates the frequency, rate or extent of androst-4-ene-3,17-dione biosynthetic process. Also known as: regulation of androst-4-ene-3,17-dione anabolism, regulation of androst-4-ene-3,17-dione biosynthesis, regulation of androst-4-ene-3,17-dione formation, regulation of androst-4-ene-3,17-dione synthesis, regulation of androstenedione biosynthetic process References: PMID:24399684 Sources: GOC:TermGenie, GOC:mr, GO_REF:0000058